symbiont-mediated perturbation of host Rab small GTPase signal transduction [GO:0141127] (biological process) Also known as: modulation by symbiont of host Rab protein mediated signal transduction, modulation by symbiont of host Rab protein signal transduction, modulation by symbiont of host Rab protein-mediated signal transduction, modulation of host Rab protein signal transduction by symbiont, modulation of host Rab protein signaling by symbiont, modulation of host Rab protein signalling by symbiont, perturbation of host Rab protein signal transduction, symbiont-mediated perturbation of host Rab protein signal transduction Relationships: is a type of symbiont-mediated perturbation of host small GTPase-mediated signal transduction [GO:0044082] References: PMID:24251537, PMID:30181274, PMID:30893609 Definition: A process in which a symbiont alters a Rab protein family-mediated signal transduction pathway in its host organism. The host is defined as the larger of the organisms involved in a symbiotic interaction.